{
  "term_id": "GO:0005543",
  "gene_symbol": "OC90",
  "gene_name": "Otoconin-90",
  "term_label": "phospholipid binding",
  "gene": "UniProtKB:Q02509"
}